rDNA spacer replication fork barrier binding, bending [GO:0110035] (molecular function) Definition: The activity of binding selectively, and in a sequence-specific manner, a replication fork barrier found in rDNA spacers, and distorting the original structure of DNA, typically a straight helix, into a bend, or increasing the bend if the original structure was intrinsically bent due to its sequence. Relationships: is a type of rDNA spacer replication fork barrier binding [GO:0043110]; is a type of GO:0044374 References: PMID:27035982 Sources: GOC:al, GOC:vw